peptidyl-serine phosphorylation [GO:0018105] (biological process) Definition: The phosphorylation of peptidyl-serine to form peptidyl-O-phospho-L-serine. Sources: RESID:AA0037 Relationships: is a type of protein phosphorylation [GO:0006468]; is_a GO:0018209 Subtypes: GO:0036289, serine phosphorylation of STAT protein [GO:0042501] Regulation: regulated by regulation of peptidyl-serine phosphorylation [GO:0033135]; negatively regulated by negative regulation of peptidyl-serine phosphorylation [GO:0033137]; RO_0002213 by GO:0033138